{
  "gene_symbol": "CYP2B6",
  "term_label": "heme binding",
  "gene": "UniProtKB:P20813",
  "gene_name": "Cytochrome P450 2B6",
  "term_id": "GO:0020037"
}